{
  "gene_symbol": "CCDC103",
  "gene": "UniProtKB:Q8IW40",
  "gene_name": "Coiled-coil domain-containing protein 103",
  "term_id": "GO:0007368",
  "term_label": "determination of left/right symmetry"
}